{
  "gene": "UniProtKB:P60900",
  "term_id": "GO:0005634",
  "gene_name": "Proteasome subunit alpha type-6",
  "term_label": "nucleus",
  "gene_symbol": "PSMA6"
}